{
  "gene_name": "Probable proton-coupled zinc antiporter SLC30A3",
  "gene": "UniProtKB:Q99726",
  "term_label": "plasma membrane",
  "gene_symbol": "SLC30A3",
  "term_id": "GO:0005886"
}